{
  "term_id": "GO:0007032",
  "gene_name": "Pleckstrin homology domain-containing family F member 2",
  "gene": "UniProtKB:Q9H8W4",
  "gene_symbol": "PLEKHF2",
  "term_label": "endosome organization"
}